actin filament [GO:0005884] (cellular component) Definition: A filamentous structure formed of a two-stranded helical polymer of the protein actin and associated proteins. Actin filaments are a major component of the contractile apparatus of skeletal muscle and the microfilaments of the cytoskeleton of eukaryotic cells. The filaments, comprising polymerized globular actin molecules, appear as flexible structures with a diameter of 5-9 nm. They are organized into a variety of linear bundles, two-dimensional networks, and three dimensional gels. In the cytoskeleton they are most highly concentrated in the cortex of the cell just beneath the plasma membrane. Subtypes: actomyosin contractile ring actin filament [GO:1903144], actin filament of cell cortex of cell tip [GO:1903145] References: PMID:10666339 Sources: GOC:mah, ISBN:0198506732 Relationships: is a type of polymeric cytoskeletal fiber [GO:0099513]; BFO_0000050 GO:0015629 Also known as: microfilament